{
  "term_label": "spindle",
  "gene": "UniProtKB:Q6IQ19",
  "gene_symbol": "CCSAP",
  "term_id": "GO:0005819",
  "gene_name": "Centriole, cilia and spindle-associated protein"
}